{
  "gene": "UniProtKB:Q14116",
  "term_id": "GO:0005125",
  "gene_name": "Interleukin-18",
  "gene_symbol": "IL18",
  "term_label": "cytokine activity"
}